chemokine receptor activity [GO:0004950] (molecular function) Definition: Combining with a chemokine, and transmitting the signal from one side of the membrane to the other to initiate a change in cell activity. Chemokines are a family of small chemotactic cytokines; their name is derived from their ability to induce directed chemotaxis in nearby responsive cells. All chemokines possess a number of conserved cysteine residues involved in intramolecular disulfide bond formation. Some chemokines are considered pro-inflammatory and can be induced during an immune response to recruit cells of the immune system to a site of infection, while others are considered homeostatic and are involved in controlling the migration of cells during normal processes of tissue maintenance or development. Chemokines are found in all vertebrates, some viruses and some bacteria. Relationships: is_a G protein-coupled chemoattractant receptor activity [GO:0001637]; is a type of cytokine receptor activity [GO:0004896]; is part of chemokine-mediated signaling pathway [GO:0070098]; has part chemokine binding [GO:0019956] References: PMID:12183377, PMID:8662823 Sources: GOC:BHF, GOC:rl, GOC:signaling, IUPHAR_GPCR:1280, Wikipedia:Chemokine Subtypes: C-C chemokine receptor activity [GO:0016493], GO:0016494, C-X3-C chemokine receptor activity [GO:0016495]